{
  "gene": "UniProtKB:Q86T24",
  "gene_name": "Transcriptional regulator Kaiso",
  "gene_symbol": "ZBTB33",
  "term_id": "GO:0000122",
  "term_label": "negative regulation of transcription by RNA polymerase II"
}